{
  "term_id": "UNKNOWN:0002",
  "term_label": "Unknown biological process",
  "gene_symbol": "CLDN25",
  "gene_name": "Putative claudin-25",
  "gene": "UniProtKB:C9JDP6"
}